{
  "term_id": "GO:0043542",
  "gene_symbol": "S100A7L2",
  "gene_name": "Protein S100-A7-like 2",
  "gene": "UniProtKB:Q5SY68",
  "term_label": "endothelial cell migration"
}